{
  "gene": "UniProtKB:P08493",
  "term_label": "extracellular matrix",
  "gene_symbol": "MGP",
  "term_id": "GO:0031012",
  "gene_name": "Matrix Gla protein"
}